{
  "gene_symbol": "KLF12",
  "term_id": "GO:0000978",
  "term_label": "RNA polymerase II cis-regulatory region sequence-specific DNA binding",
  "gene": "UniProtKB:Q9Y4X4",
  "gene_name": "Krueppel-like factor 12"
}